{
  "gene": "UniProtKB:O60673",
  "term_label": "double-strand break repair via homologous recombination",
  "gene_symbol": "REV3L",
  "term_id": "GO:0000724",
  "gene_name": "DNA polymerase zeta catalytic subunit"
}